{
  "term_id": "GO:0003684",
  "gene": "UniProtKB:Q6PJP8",
  "gene_symbol": "DCLRE1A",
  "term_label": "damaged DNA binding",
  "gene_name": "DNA cross-link repair 1A protein"
}